{
  "term_id": "GO:0005737",
  "gene_name": "Methionine-R-sulfoxide reductase B2, mitochondrial",
  "gene_symbol": "MSRB2",
  "gene": "UniProtKB:Q9Y3D2",
  "term_label": "cytoplasm"
}